thrombocyte activation [GO:0071892] (biological process) Also known as: blood coagulation, thrombocyte activation Definition: A cell activation process that occurs in thrombocytes and consists of a series of progressive, overlapping events including shape change, adhesiveness, and aggregation, which, when carried through to completion, lead to the formation of a stable hemostatic plug. Thrombocytes are nucleated cells found in non-mammalian vertebrates and are involved in hemostasis. They are the functional equivalent of the non-nucleated platelets found in mammals. References: PMID:10606877, PMID:15634265, PMID:20180901 Sources: GOC:lb, GOC:mah Relationships: is a type of cell activation [GO:0001775]; is part of blood coagulation [GO:0007596]